{
  "term_id": "GO:0045944",
  "term_label": "positive regulation of transcription by RNA polymerase II",
  "gene_symbol": "LPIN1",
  "gene_name": "Phosphatidate phosphatase LPIN1",
  "gene": "UniProtKB:Q14693"
}